{
  "gene_symbol": "STRN",
  "term_label": "neuronal cell body",
  "gene_name": "Striatin",
  "term_id": "GO:0043025",
  "gene": "UniProtKB:O43815"
}